bacterial outer membrane vesicle [GO:0061701] (cellular component) Relationships: is a type of GO:1903561 Definition: A spherical, bilayered proteolipid vesicle released from gram-negative bacterial outer membranes. References: PMID:20596524 Sources: GOC:dph, GOC:pr